{
  "term_label": "nucleus",
  "gene": "UniProtKB:P0C5Y9",
  "term_id": "GO:0005634",
  "gene_symbol": "H2AB1",
  "gene_name": "Histone H2A-Bbd type 1"
}